{
  "term_id": "GO:0005634",
  "term_label": "nucleus",
  "gene": "UniProtKB:Q7L2E3",
  "gene_symbol": "DHX30",
  "gene_name": "ATP-dependent RNA helicase DHX30"
}